{
  "term_label": "DNA-binding transcription factor activity, RNA polymerase II-specific",
  "gene_symbol": "PURB",
  "gene": "UniProtKB:Q96QR8",
  "term_id": "GO:0000981",
  "gene_name": "Transcriptional activator protein Pur-beta"
}